synaptic transmission, glutamatergic [GO:0035249] (biological process) Definition: The vesicular release of glutamate from a presynapse, across a chemical synapse, the subsequent activation of glutamate receptors at the postsynapse of a target cell (neuron, muscle, or secretory cell) and the effects of this activation on the postsynaptic membrane potential and ionic composition of the postsynaptic cytosol. This process encompasses both spontaneous and evoked release of neurotransmitter and all parts of synaptic vesicle exocytosis. Evoked transmission starts with the arrival of an action potential at the presynapse. Sources: GOC:dos Relationships: is a type of chemical synaptic transmission [GO:0007268] Also known as: glutamatergic synaptic transmission Regulation: RO_0002211 by regulation of synaptic transmission, glutamatergic [GO:0051966]; negatively regulated by negative regulation of synaptic transmission, glutamatergic [GO:0051967]; RO_0002213 by positive regulation of synaptic transmission, glutamatergic [GO:0051968]